olefinic compound catabolic process [GO:0120256] (biological process) Relationships: is a type of catabolic process [GO:0009056]; is a type of GO:0120254 Subtypes: progesterone catabolic process [GO:0006709], prenol catabolic process [GO:0016092], aldosterone catabolic process [GO:0032343], curcumin catabolic process [GO:0036040], styrene catabolic process [GO:0042207], eugenol catabolic process [GO:0042856], GO:0043451, GO:0043613, limonene catabolic process [GO:0046251], stilbene catabolic process [GO:0046272], chalcone catabolic process [GO:0046280], cinnamic acid catabolic process [GO:0046281], cinnamic acid ester catabolic process [GO:0046282], abscisic acid catabolic process [GO:0046345], helvolic acid catabolic process [GO:1900811], ferulate catabolic process [GO:1901067], funalenone catabolic process [GO:1901365], all-trans-neoxanthin catabolic process [GO:1901832], (-)-exo-alpha-bergamotene catabolic process [GO:1901939], geraniol catabolic process [GO:1903447] Definition: The chemical reactions and pathways resulting in the breakdown of an olefinic compound, any compound which contains a carbon-carbon double bond (aka C=C). Sources: GOC:krc Also known as: alkene substituted compound breakdown, alkene substituted compound catabolic process, alkene substituted compound catabolism, alkene substituted compound degradation